regulation of serine-type endopeptidase activity [GO:1900003] (biological process) Sources: GOC:TermGenie Also known as: regulation of blood coagulation factor activity Definition: Any process that modulates the frequency, rate or extent of serine-type endopeptidase activity. Subtypes: negative regulation of serine-type endopeptidase activity [GO:1900004], positive regulation of serine-type endopeptidase activity [GO:1900005] Relationships: is a type of regulation of endopeptidase activity [GO:0052548]; regulates serine-type endopeptidase activity [GO:0004252]